{
  "term_label": "G protein-coupled photoreceptor activity",
  "gene_symbol": "OPN1MW2",
  "term_id": "GO:0008020",
  "gene": "UniProtKB:P0DN77",
  "gene_name": "Medium-wave-sensitive opsin 2"
}